negative regulation of binding of sperm to zona pellucida [GO:2000360] (biological process) Definition: Any process that stops, prevents or reduces the frequency, rate or extent of binding of sperm to the zona pellucida. Sources: GOC:obol Also known as: negative regulation of ZPG binding Relationships: is a type of negative regulation of cellular process [GO:0048523]; is a type of GO:2000242; is a type of regulation of binding of sperm to zona pellucida [GO:2000359]; negatively regulates binding of sperm to zona pellucida [GO:0007339]